CMP-N-acetylneuraminate monooxygenase activity [GO:0030338] (molecular function) Also known as: CMP-N-acetylneuraminic acid hydroxylase activity, CMP-N-acetylneuraminate hydroxylase activity, CMP-Neu5Ac hydroxylase activity, cytidine monophosphoacetylneuraminate monooxygenase activity Note: Note that this was EC:1.14.13.45. Relationships: is a type of oxidoreductase activity, acting on paired donors, with incorporation or reduction of molecular oxygen, another compound as one donor, and incorporation of one atom of oxygen [GO:0016716] Sources: EC:1.14.18.2 Definition: Catalysis of the reaction: CMP-N-acetyl-beta-neuraminate + 2 Fe(II)-[cytochrome b5] + 2 H+ + O2 = CMP-N-glycoloyl-beta-neuraminate + 2 Fe(III)-[cytochrome b5] + H2O.